{
  "gene": "UniProtKB:Q13683",
  "gene_name": "Integrin alpha-7",
  "gene_symbol": "ITGA7",
  "term_id": "GO:0007229",
  "term_label": "integrin-mediated signaling pathway"
}